{
  "gene_symbol": "MIDEAS",
  "gene_name": "Mitotic deacetylase-associated SANT domain protein",
  "gene": "UniProtKB:Q6PJG2",
  "term_id": "GO:0003714",
  "term_label": "transcription corepressor activity"
}